symbiont-mediated perturbation of host synaptic transmission [GO:0044758] (biological process) Relationships: is a type of symbiont-mediated perturbation of host cellular process [GO:0044068] Definition: A process in which a symbiont alters or subverts synaptic transmission, the communication from a neuron to a target (neuron, muscle, or secretory cell) across a synapse, in its host organism. Also known as: modulation by symbiont of host synaptic transmission, regulation by symbiont of host synaptic transmission Subtypes: symbiont-mediated suppression of host synaptic transmission [GO:0044759], symbiont-mediated perturbation of host cholinergic synaptic transmission [GO:0044760] References: PMID:26487282, PMID:31075318 Sources: GOC:jl